developmental process [GO:0032502] (biological process) Relationships: is a type of biological_process [GO:0008150] Sources: GOC:isa_complete Subtypes: GO:0003006, anatomical structure morphogenesis [GO:0009653], GO:0009838, meristem initiation [GO:0010014], developmental maturation [GO:0021700], dormancy process [GO:0022611], myxococcal fruiting body development [GO:0030583], developmental induction [GO:0031128], GO:0043696, sporulation [GO:0043934], GO:0048532, anatomical structure formation involved in morphogenesis [GO:0048646], anatomical structure development [GO:0048856], cellular developmental process [GO:0048869], GO:0060033, GO:0090644, plant organ senescence [GO:0090693], GO:0097737, spore-bearing structure formation [GO:0097751], maintenance of cell number [GO:0098727], animal gross anatomical part developmental process [GO:0160108], plant gross anatomical part developmental process [GO:0160109] Also known as: development, single-organism developmental process Regulation: regulated by GO:0050793; negatively regulated by GO:0051093; positively regulated by positive regulation of developmental process [GO:0051094] Definition: A biological process whose specific outcome is the progression of an integrated living unit: an anatomical structure (which may be a subcellular structure, cell, tissue, or organ), or organism over time from an initial condition to a later condition.